neurotransmitter receptor activity involved in regulation of postsynaptic membrane potential [GO:0099529] (molecular function) Definition: Neurotransmitter receptor activity occurring in the postsynaptic membrane that is involved in regulating postsynaptic membrane potential, either directly (ionotropic receptors) or indirectly (e.g. via GPCR activation of an ion channel). Sources: GOC:dos Subtypes: GO:0099579, transmitter-gated monoatomic ion channel activity involved in regulation of postsynaptic membrane potential [GO:1904315] Relationships: is a type of postsynaptic neurotransmitter receptor activity [GO:0098960]; is part of regulation of postsynaptic membrane potential [GO:0060078]